prostacyclin receptor binding [GO:0031869] (molecular function) Sources: GOC:mah, GOC:nln Also known as: prostanoid IP receptor binding, prostacyclin receptor ligand Relationships: is a type of GO:0031862 Definition: Binding to a prostacyclin receptor.